{
  "term_id": "GO:0003700",
  "term_label": "DNA-binding transcription factor activity",
  "gene": "UniProtKB:Q6ZNH5",
  "gene_name": "Zinc finger protein 497",
  "gene_symbol": "ZNF497"
}